alpha5-beta1 integrin-fibronectin-tissue transglutaminase complex [GO:0071093] (cellular component) Also known as: ITGA5-ITGB1-FN1-TGM2 complex References: PMID:10684262 Definition: A protein complex that consists of an alpha5-beta1 integrin complex bound to fibronectin and tissue transglutaminase. Relationships: is a type of plasma membrane protein complex [GO:0098797]; is a type of GO:1902494